23S rRNA (guanine(748)-N(1))-methyltransferase activity [GO:0052912] (molecular function) Relationships: is a type of rRNA (guanine-N1-)-methyltransferase activity [GO:0008989] Definition: Catalysis of the reaction: S-adenosyl-L-methionine + guanine(748) in 23S rRNA = N(1)-methylguanine(748) in 23S rRNA + S-adenosyl-L-homocysteine. Sources: EC:2.1.1.188 Also known as: 23S rRNA m(1)G(748) methyltransferase activity